{
  "gene": "UniProtKB:Q9Y5X9",
  "term_label": "extracellular space",
  "gene_symbol": "LIPG",
  "gene_name": "Endothelial lipase",
  "term_id": "GO:0005615"
}